regulation of interleukin-9 production [GO:0032678] (biological process) Subtypes: negative regulation of interleukin-9 production [GO:0032718], positive regulation of interleukin-9 production [GO:0032758] Relationships: is a type of regulation of cytokine production [GO:0001817]; RO_0002211 interleukin-9 production [GO:0032638] Definition: Any process that modulates the frequency, rate, or extent of interleukin-9 production. Sources: GOC:mah Also known as: regulation of IL-9 production, regulation of interleukin-9 biosynthetic process